HDA1 complex [GO:0070823] (cellular component) Definition: A tetrameric histone deacetylase complex that contains a Class II deacetylase catalytic subunit. In S. cerevisiae it is composed of two Hda1p subunits along with Hda2p and Hda3p. Relationships: is a type of histone deacetylase complex [GO:0000118]; is part of chromatin [GO:0000785] References: PMID:11287668, PMID:8663039 Sources: GOC:dgf, GOC:mah